{
  "term_id": "GO:0005227",
  "gene_name": "CSC1-like protein 1",
  "term_label": "calcium-activated cation channel activity",
  "gene_symbol": "TMEM63A",
  "gene": "UniProtKB:O94886"
}